{
  "term_label": "cytoplasmic vesicle",
  "gene_symbol": "HPS4",
  "gene": "UniProtKB:Q9NQG7",
  "term_id": "GO:0031410",
  "gene_name": "BLOC-3 complex member HPS4"
}